N-acetyltaurine hydrolase activity [GO:0141215] (molecular function) Relationships: is a type of hydrolase activity, acting on ester bonds [GO:0016788] Definition: Catalysis of the reaction: N-acetyltaurine + H2O = acetate + taurine. References: PMID:39112712 Sources: RHEA:81107